{
  "term_id": "GO:0070059",
  "gene_symbol": "MAP3K5",
  "gene": "UniProtKB:Q99683",
  "term_label": "intrinsic apoptotic signaling pathway in response to endoplasmic reticulum stress",
  "gene_name": "Mitogen-activated protein kinase kinase kinase 5"
}